{
  "gene_symbol": "ATP13A2",
  "gene_name": "Polyamine-transporting ATPase 13A2",
  "term_label": "regulation of autophagosome size",
  "gene": "UniProtKB:Q9NQ11",
  "term_id": "GO:0016243"
}